protein-hormone receptor activity [GO:0016500] (molecular function) Subtypes: follicle-stimulating hormone receptor activity [GO:0004963], luteinizing hormone receptor activity [GO:0004964], gonadotropin-releasing hormone receptor activity [GO:0004968], thyroid-stimulating hormone receptor activity [GO:0004996], insulin receptor activity [GO:0005009], melanin-concentrating hormone receptor activity [GO:0030273], GO:0035472, adipokinetic hormone receptor activity [GO:0097003], anti-Mullerian hormone receptor activity [GO:1990272] Sources: GOC:mah Relationships: is a type of signaling receptor activity [GO:0038023] Definition: Combining with a protein hormone to initiate a change in cell activity.